cap snatching [GO:0075526] (biological process) Sources: GOC:bf, GOC:jl, VZ:839 Relationships: is a type of viral process [GO:0016032]; is part of GO:0039697 Definition: A transcription initiation process during which a nucleotide sequence between 10 and 20 nucleotides in size is cleaved from the 5' end of host mRNAs by a viral RNA-dependent polymerase. The capped leader sequence obtained is subsequently used to prime transcription on the viral genome, which ultimately leads to the synthesis of capped, translatable viral mRNAs. Also known as: cap snatching involved in viral mRNA transcription